positive regulation of intermediate filament depolymerization [GO:0030844] (biological process) Definition: Any process that activates or increases the frequency, rate or extent of intermediate filament depolymerization. Note: Note that this term was split from 'positive regulation of intermediate filament polymerization and/or depolymerization ; GO:0045826' (sibling term 'positive regulation of intermediate filament polymerization ; GO:0030841'). Also known as: positive regulation of intermediate filament polymerization and/or depolymerization, up regulation of intermediate filament depolymerization, up-regulation of intermediate filament depolymerization, upregulation of intermediate filament depolymerization, activation of intermediate filament depolymerization, stimulation of intermediate filament depolymerization Sources: GOC:mah Relationships: is a type of regulation of intermediate filament depolymerization [GO:0030842]; is a type of positive regulation of cytoskeleton organization [GO:0051495]; is a type of positive regulation of protein depolymerization [GO:1901881]; positively regulates GO:0045106